{
  "gene_name": "Zinc finger protein 544",
  "term_id": "GO:0000976",
  "term_label": "transcription cis-regulatory region binding",
  "gene": "UniProtKB:Q6NX49",
  "gene_symbol": "ZNF544"
}